ribose phosphate biosynthetic process [GO:0046390] (biological process) Relationships: is a type of ribose phosphate metabolic process [GO:0019693]; is a type of organophosphate biosynthetic process [GO:0090407]; is a type of carbohydrate derivative biosynthetic process [GO:1901137] Definition: The chemical reactions and pathways resulting in the formation of ribose phosphate, any phosphorylated ribose sugar. Subtypes: GO:0006015, ribonucleotide biosynthetic process [GO:0009260], D-ribose 5-phosphate biosynthetic process [GO:1901280] Sources: GOC:ai Also known as: ribose phosphate anabolism, ribose phosphate biosynthesis, ribose phosphate formation, ribose phosphate synthesis